response to virus [GO:0009615] (biological process) Sources: GOC:hb Definition: Any process that results in a change in state or activity of a cell or an organism (in terms of movement, secretion, enzyme production, gene expression, etc.) as a result of a stimulus from a virus. Subtypes: detection of virus [GO:0009597], GO:0039634, defense response to virus [GO:0051607], cellular response to virus [GO:0098586] Also known as: response to viruses Relationships: is_a response to other organism [GO:0051707]